regulation of plasma kallikrein-kinin cascade [GO:0002529] (biological process) Relationships: is a type of regulation of kinin cascade [GO:0002256]; regulates plasma kallikrein-kinin cascade [GO:0002353] Sources: GOC:add Definition: Any process that modulates the frequency, rate, or extent of the plasma kallikrein-kinin cascade. Subtypes: negative regulation of plasma kallikrein-kinin cascade [GO:0002549], positive regulation of plasma kallikrein-kinin cascade [GO:0002550]